response to external stimulus [GO:0009605] (biological process) Regulation: RO_0002211 by regulation of response to external stimulus [GO:0032101]; negatively regulated by negative regulation of response to external stimulus [GO:0032102]; positively regulated by GO:0032103 Relationships: is a type of response to stimulus [GO:0050896] Subtypes: startle response [GO:0001964], detection of external stimulus [GO:0009581], tropism [GO:0009606], GO:0009612, entrainment of circadian clock [GO:0009649], GO:0042465, GO:0043207, pigment accumulation [GO:0043476], polyphenic determination, influence by environmental factors [GO:0048651], GO:0060004, cellular response to external stimulus [GO:0071496], response to environmental enrichment [GO:0090648] Sources: GOC:hb Definition: Any process that results in a change in state or activity of a cell or an organism (in terms of movement, secretion, enzyme production, gene expression, etc.) as a result of an external stimulus. Note: Note that this term is in the subset of terms that should not be used for direct gene product annotation. Instead, select a child term or, if no appropriate child term exists, please request a new term. Direct annotations to this term may be amended during annotation QC. Also known as: response to environmental stimulus